S-adenosylmethioninamine metabolic process [GO:0046499] (biological process) Definition: The chemical reactions and pathways involving S-adenosylmethioninamine, (5-deoxy-5-adenosyl)(3-aminopropyl) methylsulfonium salt. Relationships: is a type of sulfur compound metabolic process [GO:0006790]; is_a purine ribonucleoside metabolic process [GO:0046128] Also known as: S-adenosylmethioninamine metabolism Sources: GOC:mah